{
  "term_id": "GO:0003682",
  "gene": "UniProtKB:Q8IXJ9",
  "term_label": "chromatin binding",
  "gene_symbol": "ASXL1",
  "gene_name": "Polycomb group protein ASXL1"
}